{
  "gene_symbol": "MANSC1",
  "gene_name": "MANSC domain-containing protein 1",
  "term_id": "UNKNOWN:0001",
  "gene": "UniProtKB:Q9H8J5",
  "term_label": "Unknown molecular function"
}